{
  "gene_symbol": "SERPINA11",
  "term_label": "Unknown biological process",
  "term_id": "UNKNOWN:0002",
  "gene": "UniProtKB:Q86U17",
  "gene_name": "Serpin A11"
}